{
  "gene": "UniProtKB:P36575",
  "term_id": "GO:0007601",
  "gene_symbol": "ARR3",
  "term_label": "visual perception",
  "gene_name": "Arrestin-C"
}